{
  "gene": "UniProtKB:P25800",
  "gene_symbol": "LMO1",
  "term_id": "GO:0005634",
  "gene_name": "Rhombotin-1",
  "term_label": "nucleus"
}